{
  "term_label": "nucleoplasm",
  "gene": "UniProtKB:P29728",
  "term_id": "GO:0005654",
  "gene_name": "2'-5'-oligoadenylate synthase 2",
  "gene_symbol": "OAS2"
}